{
  "term_label": "ciliary transition zone",
  "term_id": "GO:0035869",
  "gene_symbol": "TMEM231",
  "gene_name": "Transmembrane protein 231",
  "gene": "UniProtKB:Q9H6L2"
}